{
  "gene_name": "Cold shock domain-containing protein E1",
  "gene": "UniProtKB:O75534",
  "gene_symbol": "CSDE1",
  "term_id": "GO:0140517",
  "term_label": "protein-RNA adaptor activity"
}